mitochondrial tRNA wobble position uridine thiolation [GO:1990799] (biological process) References: PMID:15509579 Definition: The process in which a uridine residue at position 34 in the anticodon of a mitochondrial tRNA is post-transcriptionally thiolated at the C2 position. This process involves transfer of a sulfur from cysteine to position C2 by several steps. Relationships: is_a GO:0002143; is_a mitochondrial tRNA wobble uridine modification [GO:0070899]; is a type of mitochondrial tRNA thio-modification [GO:0070903]